GTP binding [GO:0005525] (molecular function) Sources: GOC:ai Relationships: is a type of GO:0032561; is a type of purine ribonucleoside triphosphate binding [GO:0035639] Regulation: positively regulated by guanyl-nucleotide exchange factor activity [GO:0005085]; positively regulated by positive regulation of GTP binding [GO:1904426] Definition: Binding to GTP, guanosine triphosphate.